{
  "term_label": "plasma membrane",
  "gene": "UniProtKB:Q9NQ75",
  "term_id": "GO:0005886",
  "gene_name": "Cas scaffolding protein family member 4",
  "gene_symbol": "CASS4"
}